{
  "gene_symbol": "ROR2",
  "term_label": "transmembrane receptor protein tyrosine kinase activity",
  "gene": "UniProtKB:Q01974",
  "term_id": "GO:0004714",
  "gene_name": "Tyrosine-protein kinase transmembrane receptor ROR2"
}